carnitine transmembrane transport [GO:1902603] (biological process) Definition: The directed movement of carnitine across a membrane. Sources: GOC:TermGenie, GOC:pr, GO_REF:0000069 Subtypes: (R)-carnitine transmembrane transport [GO:1902270] Relationships: is a type of carnitine transport [GO:0015879]; is a type of GO:0055085